{
  "gene": "UniProtKB:Q9BZA7",
  "gene_symbol": "PCDH11X",
  "gene_name": "Protocadherin-11 X-linked",
  "term_id": "GO:0005886",
  "term_label": "plasma membrane"
}